{
  "gene": "UniProtKB:Q7Z401",
  "term_id": "GO:0032483",
  "term_label": "regulation of Rab protein signal transduction",
  "gene_name": "C-myc promoter-binding protein",
  "gene_symbol": "DENND4A"
}